{
  "gene_symbol": "PRKACB",
  "gene": "UniProtKB:P22694",
  "term_id": "GO:0005829",
  "gene_name": "cAMP-dependent protein kinase catalytic subunit beta",
  "term_label": "cytosol"
}